{
  "gene_name": "Vasopressin V1b receptor",
  "gene": "UniProtKB:P47901",
  "term_id": "GO:0001992",
  "gene_symbol": "AVPR1B",
  "term_label": "regulation of systemic arterial blood pressure by vasopressin"
}